rhoptry [GO:0020008] (cellular component) Relationships: is_a cellular anatomical structure [GO:0110165]; is part of apical complex [GO:0020007] Definition: A large, club-shaped secretory organelle that forms part of the apical complex of an apicomplexan parasite, and consists of a bulbous body and a narrow electron-dense neck that extends through the conoid at the apical tip of the parasite. The rhoptry necks serve as ducts through which the contents of the rhoptries are secreted after attachment to the host has been completed and at the commencement of invasion. Rhoptry proteins function in the biogenesis and host organellar association of the parasitophorous vacuole. Also known as: paired organelles, toxoneme References: PMID:11801218, PMID:16002398 Sources: ISBN:0521664470